{
  "term_id": "GO:0010468",
  "gene_name": "Probable lysine-specific demethylase 4F",
  "gene_symbol": "KDM4F",
  "gene": "UniProtKB:A0A1W2PPD8",
  "term_label": "regulation of gene expression"
}